{
  "gene_name": "Elongation of very long chain fatty acids protein 3",
  "gene": "UniProtKB:Q9HB03",
  "term_id": "GO:0042761",
  "gene_symbol": "ELOVL3",
  "term_label": "very long-chain fatty acid biosynthetic process"
}